{
  "term_id": "GO:0017025",
  "gene": "UniProtKB:P52657",
  "gene_symbol": "GTF2A2",
  "gene_name": "Transcription initiation factor IIA subunit 2",
  "term_label": "TBP-class protein binding"
}